{
  "gene": "UniProtKB:P46781",
  "gene_symbol": "RPS9",
  "term_label": "rRNA binding",
  "term_id": "GO:0019843",
  "gene_name": "Small ribosomal subunit protein uS4"
}